{
  "term_label": "Unknown molecular function",
  "gene_symbol": "CLDN4",
  "gene": "UniProtKB:O14493",
  "term_id": "UNKNOWN:0001",
  "gene_name": "Claudin-4"
}